{
  "term_id": "GO:0005852",
  "term_label": "eukaryotic translation initiation factor 3 complex",
  "gene": "UniProtKB:Q7L2H7",
  "gene_name": "Eukaryotic translation initiation factor 3 subunit M",
  "gene_symbol": "EIF3M"
}